{
  "gene_symbol": "HEPH",
  "term_label": "Unknown biological process",
  "gene": "UniProtKB:Q9BQS7",
  "gene_name": "Hephaestin",
  "term_id": "UNKNOWN:0002"
}